{
  "gene_name": "Protein JTB",
  "term_label": "midbody",
  "gene_symbol": "JTB",
  "term_id": "GO:0030496",
  "gene": "UniProtKB:O76095"
}